{
  "gene": "UniProtKB:Q8TBZ5",
  "term_label": "regulation of DNA-templated transcription",
  "term_id": "GO:0006355",
  "gene_name": "Zinc finger protein 502",
  "gene_symbol": "ZNF502"
}